phosphatidylinositol-4,5-bisphosphate binding [GO:0005546] (MF) Also known as: PIP2 binding, 1-phosphatidyl-1D-myo-inositol 4,5-bisphosphate binding, PtdIns(4,5)P2 binding, phosphatidylinositol 4,5-bisphosphate binding Sources: GOC:bf, GOC:jl Definition: Binding to phosphatidylinositol-4,5-bisphosphate, a derivative of phosphatidylinositol in which the inositol ring is phosphorylated at the 4' and 5' positions. Relationships: is a type of anion binding [GO:0043168]; is a type of phosphatidylinositol bisphosphate binding [GO:1902936]